{
  "gene": "UniProtKB:O60895",
  "term_id": "GO:0032870",
  "gene_symbol": "RAMP2",
  "term_label": "cellular response to hormone stimulus",
  "gene_name": "Receptor activity-modifying protein 2"
}